{
  "term_id": "GO:0000978",
  "gene_name": "Endothelial zinc finger protein induced by tumor necrosis factor alpha",
  "gene_symbol": "ZNF71",
  "gene": "UniProtKB:Q9NQZ8",
  "term_label": "RNA polymerase II cis-regulatory region sequence-specific DNA binding"
}